{
  "gene_name": "RNA-splicing ligase RtcB homolog",
  "gene": "UniProtKB:Q9Y3I0",
  "term_id": "GO:0005634",
  "gene_symbol": "RTCB",
  "term_label": "nucleus"
}